{
  "gene": "UniProtKB:Q9NPC1",
  "term_id": "GO:0008528",
  "gene_name": "Leukotriene B4 receptor 2",
  "term_label": "G protein-coupled peptide receptor activity",
  "gene_symbol": "LTB4R2"
}